{
  "gene_name": "Abasic site processing protein HMCES",
  "gene_symbol": "HMCES",
  "term_id": "GO:0106300",
  "term_label": "protein-DNA covalent cross-linking repair",
  "gene": "UniProtKB:Q96FZ2"
}